{
  "gene_symbol": "AGK",
  "gene": "UniProtKB:Q53H12",
  "term_id": "GO:0005886",
  "term_label": "plasma membrane",
  "gene_name": "Acylglycerol kinase, mitochondrial"
}